positive regulation of ecdysone receptor signaling pathway [GO:0120142] (biological process) Relationships: is a type of positive regulation of intracellular steroid hormone receptor signaling pathway [GO:0033145]; is a type of GO:0120141; positively regulates ecdysone receptor signaling pathway [GO:0035076] Definition: Any process that activates or increases the frequency, rate or extent of any ecdysone receptor signaling pathway. References: PMID:23072462 Sources: GOC:ha Also known as: positive regulation of ecdysone receptor-mediated signaling pathway